guard mother cell cytokinesis [GO:0010235] (biological process) Also known as: guard mother cell division Sources: GOC:tb Relationships: is a type of cytokinesis by cell plate formation [GO:0000911]; is part of stomatal lineage progression [GO:0010440] Definition: The stereotyped symmetric cell division by which guard mother cell give rise to stomatal guard cells.